{
  "gene": "UniProtKB:Q8NEL0",
  "term_id": "UNKNOWN:0003",
  "term_label": "Unknown cellular component",
  "gene_name": "Coiled-coil domain-containing protein 54",
  "gene_symbol": "CCDC54"
}